heme C biosynthetic process [GO:0006786] (BP) Relationships: is_a GO:0006783 Sources: GOC:curators, PubChem_Compound:122208 Also known as: haem C biosynthesis, haem C biosynthetic process, heme C anabolism, heme C biosynthesis, heme C formation, heme C synthesis Definition: The chemical reactions and pathways resulting in the formation of heme c, a derivative of heme found in cytochromes c, b4, and f.